{
  "term_id": "GO:0005634",
  "gene_name": "Zinc finger protein 841",
  "gene_symbol": "ZNF841",
  "gene": "UniProtKB:Q6ZN19",
  "term_label": "nucleus"
}